{
  "gene_symbol": "PARP1",
  "term_id": "GO:0140807",
  "gene": "UniProtKB:P09874",
  "gene_name": "Poly [ADP-ribose] polymerase 1",
  "term_label": "NAD+-protein-glutamate ADP-ribosyltransferase activity"
}